{
  "term_label": "ciliary base",
  "gene_name": "Sperm acrosome-associated protein 9",
  "term_id": "GO:0097546",
  "gene_symbol": "SPACA9",
  "gene": "UniProtKB:Q96E40"
}